{
  "gene": "UniProtKB:Q9H898",
  "term_id": "UNKNOWN:0001",
  "gene_symbol": "ZMAT4",
  "term_label": "Unknown molecular function",
  "gene_name": "Zinc finger matrin-type protein 4"
}